{
  "gene_symbol": "CHMP6",
  "term_label": "late endosome to vacuole transport via multivesicular body sorting pathway",
  "gene": "UniProtKB:Q96FZ7",
  "gene_name": "Charged multivesicular body protein 6",
  "term_id": "GO:0032511"
}